{
  "gene": "UniProtKB:P0C5J1",
  "gene_name": "Putative protein N-methyltransferase FAM86B2",
  "term_id": "GO:0016279",
  "gene_symbol": "FAM86B2",
  "term_label": "protein-lysine N-methyltransferase activity"
}